{
  "gene_name": "Heat shock protein beta-6",
  "term_label": "protein refolding",
  "gene_symbol": "HSPB6",
  "term_id": "GO:0042026",
  "gene": "UniProtKB:O14558"
}